negative regulation of vascular associated smooth muscle contraction [GO:1904694] (biological process) Relationships: is a type of regulation of vascular associated smooth muscle contraction [GO:0003056]; is a type of negative regulation of vasoconstriction [GO:0045906]; is a type of GO:0045986; negatively regulates vascular associated smooth muscle contraction [GO:0014829] Also known as: down regulation of vascular smooth muscle contraction, down-regulation of vascular smooth muscle contraction, downregulation of vascular smooth muscle contraction, negative regulation of vascular smooth muscle contraction, inhibition of vascular smooth muscle contraction Subtypes: GO:0062088, GO:1905655 Definition: Any process that stops, prevents or reduces the frequency, rate or extent of vascular smooth muscle contraction. References: PMID:22158624 Sources: GOC:BHF, GOC:BHF_miRNA, GOC:TermGenie, GOC:rph, GO_REF:0000058